{
  "gene_symbol": "TRAJ27",
  "gene_name": "T cell receptor alpha joining 27 (Fragment)",
  "gene": "UniProtKB:A0A075B6W6",
  "term_label": "Unknown molecular function",
  "term_id": "UNKNOWN:0001"
}